{
  "gene_symbol": "CDCP1",
  "term_label": "Unknown molecular function",
  "gene": "UniProtKB:Q9H5V8",
  "term_id": "UNKNOWN:0001",
  "gene_name": "CUB domain-containing protein 1"
}